{
  "term_id": "UNKNOWN:0003",
  "gene_name": "Protein PMS2CL",
  "term_label": "Unknown cellular component",
  "gene_symbol": "PMS2CL",
  "gene": "UniProtKB:Q68D20"
}